{
  "gene": "UniProtKB:P22003",
  "term_label": "cytokine activity",
  "gene_symbol": "BMP5",
  "term_id": "GO:0005125",
  "gene_name": "Bone morphogenetic protein 5"
}